{
  "term_id": "GO:0071805",
  "gene": "UniProtKB:Q92953",
  "gene_name": "Potassium voltage-gated channel subfamily B member 2",
  "term_label": "potassium ion transmembrane transport",
  "gene_symbol": "KCNB2"
}